{
  "gene": "UniProtKB:Q9Y5X2",
  "gene_name": "Sorting nexin-8",
  "gene_symbol": "SNX8",
  "term_id": "GO:0034498",
  "term_label": "early endosome to Golgi transport"
}